{
  "term_id": "GO:0006357",
  "gene_symbol": "PRDM16",
  "gene_name": "Histone-lysine N-methyltransferase PRDM16",
  "gene": "UniProtKB:Q9HAZ2",
  "term_label": "regulation of transcription by RNA polymerase II"
}